{
  "gene": "UniProtKB:Q8N8J7",
  "gene_symbol": "FAM241A",
  "term_id": "UNKNOWN:0002",
  "gene_name": "Uncharacterized protein FAM241A",
  "term_label": "Unknown biological process"
}